positive regulation of gap junction assembly [GO:1903598] (biological process) Also known as: up regulation of gap junction assembly, up-regulation of gap junction assembly, upregulation of gap junction assembly, activation of gap junction assembly Definition: Any process that activates or increases the frequency, rate or extent of gap junction assembly. Relationships: is a type of positive regulation of cell junction assembly [GO:1901890]; is a type of regulation of gap junction assembly [GO:1903596]; positively regulates gap junction assembly [GO:0016264] References: PMID:25017399 Sources: GOC:BHF, GOC:TermGenie, GOC:mtg_cardiac_conduct_nov11, GOC:rl, GO_REF:0000058